{
  "gene_symbol": "TAF11L5",
  "term_id": "GO:0051123",
  "term_label": "RNA polymerase II preinitiation complex assembly",
  "gene_name": "TATA-box-binding protein-associated factor 11-like protein 5",
  "gene": "UniProtKB:A0A1W2PP81"
}